UDP-galactose transmembrane transport [GO:0072334] (biological process) Note: Note that this term is not intended for use in annotating lateral movement within membranes. Subtypes: UDP-galactose transmembrane import into Golgi lumen [GO:0097624] Definition: The process in which UDP-galactose is transported across a membrane. Also known as: UDP-galactose membrane transport, UDP-galactose transport Relationships: is_a organic anion transport [GO:0015711]; is a type of pyrimidine nucleotide-sugar transmembrane transport [GO:0090481] Sources: GOC:mah